{
  "gene_name": "Putative HERC2-like protein 3",
  "gene_symbol": "HERC2P3",
  "term_label": "cytoplasm",
  "term_id": "GO:0005737",
  "gene": "UniProtKB:Q9BVR0"
}